{
  "term_id": "GO:0032816",
  "gene_symbol": "TYROBP",
  "term_label": "positive regulation of natural killer cell activation",
  "gene_name": "TYRO protein tyrosine kinase-binding protein",
  "gene": "UniProtKB:O43914"
}